{
  "term_id": "GO:0007399",
  "term_label": "nervous system development",
  "gene_name": "RNA binding protein fox-1 homolog 2",
  "gene": "UniProtKB:O43251",
  "gene_symbol": "RBFOX2"
}